organellar chromatophore thylakoid lumen [GO:0070117] (cellular component) Relationships: is a type of thylakoid lumen [GO:0031977]; is part of organellar chromatophore thylakoid [GO:0070116] Also known as: Paulinella-type chromatophore thylakoid lumen Definition: The volume enclosed by an organellar chromatophore thylakoid membrane. Sources: GOC:mah